{
  "gene_name": "Cardiomyopathy-associated protein 5",
  "term_label": "cytoplasm",
  "gene_symbol": "CMYA5",
  "term_id": "GO:0005737",
  "gene": "UniProtKB:Q8N3K9"
}